{
  "gene_symbol": "RAD23B",
  "term_id": "GO:0031593",
  "gene_name": "UV excision repair protein RAD23 homolog B",
  "gene": "UniProtKB:P54727",
  "term_label": "polyubiquitin modification-dependent protein binding"
}